{
  "term_id": "GO:0032486",
  "gene_name": "Ras-related protein Rap-1A",
  "term_label": "Rap protein signal transduction",
  "gene": "UniProtKB:P62834",
  "gene_symbol": "RAP1A"
}